{
  "gene_symbol": "FAM171A2",
  "term_id": "UNKNOWN:0002",
  "gene_name": "Protein FAM171A2",
  "term_label": "Unknown biological process",
  "gene": "UniProtKB:A8MVW0"
}